{
  "term_id": "GO:0005657",
  "gene_name": "DNA repair protein RAD51 homolog 4",
  "gene": "UniProtKB:O75771",
  "term_label": "replication fork",
  "gene_symbol": "RAD51D"
}